{
  "term_label": "RNA polymerase II cis-regulatory region sequence-specific DNA binding",
  "gene_name": "Forkhead box protein O1",
  "gene": "UniProtKB:Q12778",
  "term_id": "GO:0000978",
  "gene_symbol": "FOXO1"
}